rhombomere 2 morphogenesis [GO:0021655] (biological process) Sources: GOC:cls, GOC:curators, GOC:dgh, GOC:dph, GOC:jid Definition: The process in which the anatomical structure of rhombomere 2 is generated and organized. Rhombomeres are transverse segments of the developing rhombencephalon. Rhombomeres are lineage restricted, express different genes from one another, and adopt different developmental fates. Rhombomeres are numbered in an anterior to posterior order. Relationships: is a type of GO:0021593; is part of GO:0021568